{
  "term_label": "regulation of synaptic assembly at neuromuscular junction",
  "gene_name": "PDZ domain-containing protein 11",
  "gene": "UniProtKB:Q5EBL8",
  "term_id": "GO:0008582",
  "gene_symbol": "PDZD11"
}